{
  "term_id": "UNKNOWN:0001",
  "term_label": "Unknown molecular function",
  "gene_symbol": "SH2D1B",
  "gene": "UniProtKB:O14796",
  "gene_name": "SH2 domain-containing protein 1B"
}